{
  "term_id": "GO:0005886",
  "term_label": "plasma membrane",
  "gene": "UniProtKB:Q9NS86",
  "gene_symbol": "LANCL2",
  "gene_name": "LanC-like protein 2"
}